host outer membrane [GO:0044384] (cellular component) Subtypes: host organelle outer membrane [GO:0039661], host cell outer membrane [GO:0039662] Sources: GOC:jl Note: This term covers the outer membrane of the host cell envelope or the outer membrane of a host organelle. For the outer layer of the host cell envelope specifically, see host cell outer membrane ; GO:0039662. Definition: The external membrane of Gram-negative bacteria or certain organelles such as mitochondria and chloroplasts; freely permeable to most ions and metabolites, occurring in a host cell. Relationships: is a type of host cell membrane [GO:0033644] Also known as: host cell outer membrane